{
  "gene": "UniProtKB:Q6ZRT6",
  "gene_name": "Proline-rich protein 23B",
  "gene_symbol": "PRR23B",
  "term_label": "Unknown molecular function",
  "term_id": "UNKNOWN:0001"
}